{
  "gene": "UniProtKB:O14841",
  "gene_name": "5-oxoprolinase",
  "term_id": "GO:0006749",
  "gene_symbol": "OPLAH",
  "term_label": "glutathione metabolic process"
}